{
  "term_label": "regulation of transcription by RNA polymerase II",
  "term_id": "GO:0006357",
  "gene_name": "Forkhead box protein I1",
  "gene_symbol": "FOXI1",
  "gene": "UniProtKB:Q12951"
}